{
  "gene_symbol": "MYOCD",
  "term_label": "positive regulation of transcription by RNA polymerase II",
  "gene_name": "Myocardin",
  "gene": "UniProtKB:Q8IZQ8",
  "term_id": "GO:0045944"
}